{
  "gene_symbol": "GPR4",
  "gene": "UniProtKB:P46093",
  "term_label": "adenylate cyclase-activating G protein-coupled receptor signaling pathway",
  "term_id": "GO:0007189",
  "gene_name": "G-protein coupled receptor 4"
}